{
  "gene": "UniProtKB:Q5XG85",
  "gene_symbol": "Q5XG85",
  "term_label": "Unknown biological process",
  "term_id": "UNKNOWN:0002",
  "gene_name": "Putative UPF0633 protein LOC554249"
}